collagen type XVI trimer [GO:0005597] (cellular component) Relationships: is a type of FACIT collagen trimer [GO:0005593] References: PMID:12782140 Definition: A collagen trimer containing alpha(XVI) chains; type XVI trimers can associate with microfibrils.